{
  "term_label": "Unknown biological process",
  "term_id": "UNKNOWN:0002",
  "gene": "UniProtKB:Q5H9R4",
  "gene_name": "Armadillo repeat-containing X-linked protein 4",
  "gene_symbol": "ARMCX4"
}